{
  "gene_symbol": "STMN4",
  "term_label": "microtubule depolymerization",
  "term_id": "GO:0007019",
  "gene": "UniProtKB:Q9H169",
  "gene_name": "Stathmin-4"
}